{
  "gene_symbol": "TIGIT",
  "term_id": "GO:0005102",
  "gene": "UniProtKB:Q495A1",
  "gene_name": "T-cell immunoreceptor with Ig and ITIM domains",
  "term_label": "signaling receptor binding"
}